{
  "gene_name": "Probable methyltransferase-like protein 25",
  "gene": "UniProtKB:Q8N6Q8",
  "term_id": "UNKNOWN:0003",
  "term_label": "Unknown cellular component",
  "gene_symbol": "METTL25"
}